{
  "term_label": "spliceosomal complex",
  "gene_name": "Beta-catenin-like protein 1",
  "term_id": "GO:0005681",
  "gene_symbol": "CTNNBL1",
  "gene": "UniProtKB:Q8WYA6"
}